negative regulation of establishment of protein localization [GO:1904950] (biological process) References: PMID:22761445 Sources: GOC:TermGenie, GO_REF:0000058 Also known as: down regulation of establishment of protein localisation, down regulation of establishment of protein localization, down regulation of protein positioning, down regulation of protein recruitment, down-regulation of establishment of protein localisation, down-regulation of establishment of protein localization, down-regulation of protein positioning, down-regulation of protein recruitment, downregulation of establishment of protein localisation, downregulation of establishment of protein localization, downregulation of protein positioning, downregulation of protein recruitment, negative regulation of establishment of protein localisation, negative regulation of protein positioning, negative regulation of protein recruitment, inhibition of establishment of protein localisation, inhibition of establishment of protein localization, inhibition of protein positioning, inhibition of protein recruitment Relationships: is a type of negative regulation of biological process [GO:0048519]; is a type of regulation of establishment of protein localization [GO:0070201]; negatively regulates establishment of protein localization [GO:0045184] Definition: Any process that stops, prevents or reduces the frequency, rate or extent of establishment of protein localization. Subtypes: negative regulation of protein transport [GO:0051224], negative regulation of protein targeting to membrane [GO:0090315], GO:1903748, GO:1904850